{
  "term_id": "GO:0043161",
  "term_label": "proteasome-mediated ubiquitin-dependent protein catabolic process",
  "gene_symbol": "WWP2",
  "gene": "UniProtKB:O00308",
  "gene_name": "NEDD4-like E3 ubiquitin-protein ligase WWP2"
}